{
  "gene_symbol": "ASIC3",
  "gene": "UniProtKB:Q9UHC3",
  "gene_name": "Acid-sensing ion channel 3",
  "term_id": "GO:0005886",
  "term_label": "plasma membrane"
}